{
  "gene_symbol": "MUC7",
  "gene": "UniProtKB:Q8TAX7",
  "term_id": "UNKNOWN:0001",
  "term_label": "Unknown molecular function",
  "gene_name": "Mucin-7"
}